{
  "gene": "UniProtKB:Q49AJ0",
  "term_id": "UNKNOWN:0001",
  "term_label": "Unknown molecular function",
  "gene_symbol": "FAM135B",
  "gene_name": "Protein FAM135B"
}